{
  "gene_name": "Matrix Gla protein",
  "gene": "UniProtKB:P08493",
  "term_label": "Unknown biological process",
  "gene_symbol": "MGP",
  "term_id": "UNKNOWN:0002"
}